inner ear auditory receptor cell differentiation [GO:0042491] (BP) Definition: The process in which a relatively unspecialized inner cell acquires specialized features of an auditory hair cell. Sources: CL:0000201, GOC:jl Also known as: auditory hair cell differentiation, auditory receptor cell differentiation Regulation: regulated by GO:0045607; negatively regulated by GO:0045608; positively regulated by GO:0045609 Relationships: is a type of hair cell differentiation [GO:0035315]; is a type of GO:0060113 Note: Note that this term refers to the mechanosensory hair cells of the inner ear.